epidermal growth factor receptor ligand maturation [GO:0038004] (biological process) References: PMID:11672524, PMID:11672525 Sources: GOC:signaling Definition: Any process leading to the attainment of the full functional capacity of a ligand for an epidermal growth factor receptor. The ligand is functional when it can bind to and activate an epidermal growth factor receptor. Relationships: is a type of peptide hormone processing [GO:0016486]; BFO_0000051 membrane protein ectodomain proteolysis [GO:0006509] Also known as: EGFR ligand maturation, EGFR ligand maturation by peptide bond cleavage, EGFR ligand processing, peptide bond cleavage involved in EGFR ligand maturation, epidermal growth factor receptor ligand processing, peptide bond cleavage involved in epidermal growth factor receptor ligand maturation